GAG codon-amino acid adaptor activity [GO:0033460] (molecular function) Definition: A triplet codon-amino acid adaptor activity that recognizes a GAG codon. Sources: GOC:mah Also known as: glutamic acid tRNA Note: Note that in the standard genetic code, GAG codes for glutamic acid. Relationships: is a type of GO:0030533